negative regulation of dehydroepiandrosterone secretion [GO:2000841] (biological process) Also known as: negative regulation of 3beta-hydroxyandrost-5-en-17-one secretion, negative regulation of DHEA secretion, negative regulation of dehydroisoandrosterone secretion Sources: GOC:sl Definition: Any process that stops, prevents or reduces the frequency, rate or extent of dehydroepiandrosterone secretion. Relationships: is a type of negative regulation of lipid transport [GO:0032369]; is a type of negative regulation of hormone secretion [GO:0046888]; is_a regulation of dehydroepiandrosterone secretion [GO:2000840]; negatively regulates dehydroepiandrosterone secretion [GO:0035942]